{
  "term_label": "Unknown biological process",
  "gene_name": "Centrosomal AT-AC splicing factor",
  "gene": "UniProtKB:Q86UT8",
  "term_id": "UNKNOWN:0002",
  "gene_symbol": "CENATAC"
}